{
  "gene": "UniProtKB:P80075",
  "gene_symbol": "CCL8",
  "term_id": "GO:0006954",
  "term_label": "inflammatory response",
  "gene_name": "C-C motif chemokine 8"
}